{
  "gene_name": "Neurexin-1",
  "gene": "UniProtKB:Q9ULB1",
  "term_id": "GO:0048787",
  "gene_symbol": "NRXN1",
  "term_label": "presynaptic active zone membrane"
}